arabinose isomerase activity [GO:0008790] (molecular function) Definition: Catalysis of the reaction: D-arabinose = D-ribulose. Sources: EC:5.3.1.3 Also known as: D-arabinose isomerase activity, D-arabinose aldose-ketose-isomerase activity, D-arabinose ketol-isomerase activity, D-arabinose(L-fucose) isomerase activity Relationships: is a type of intramolecular oxidoreductase activity, interconverting aldoses and ketoses [GO:0016861]